spliceosomal tri-snRNP complex assembly [GO:0000244] (biological process) Relationships: is a type of spliceosomal snRNP assembly [GO:0000387] Definition: The formation of a tri-snRNP complex containing U4 and U6 (or U4atac and U6atac) snRNAs and U5 snRNAs and associated proteins. This includes reannealing of U4 and U6 (or U4atac and U6atac) snRNAs released from previous rounds of splicing to reform the U4/U6 snRNP (or U4atac/U6atac snRNP) as well as the subsequent association of the U5 snRNP with the U4/U6 snRNP (or U4atac/U6atac snRNP) to form a tri-snRNP that is ready to reassemble into another spliceosome complex. References: PMID:9452384 Sources: ISBN:0879695897 Also known as: snRNP recycling, assembly of spliceosomal tri-snRNP, spliceosomal tri-snRNP assembly, assembly of spliceosomal tri-snRNP U4/U6.U5, assembly of spliceosomal tri-snRNP U4atac/U6atac.U5, spliceosomal tri-snRNP U4/U6.U5 assembly, spliceosomal tri-snRNP U4atac/U6atac.U5 assembly